phosphatidylinositol kinase activity [GO:0052742] (molecular function) Definition: Catalysis of the reaction: ATP + a phosphatidylinositol = ADP + a phosphatidylinositol phosphate. Sources: GOC:ai Also known as: 1-phosphatidylinositol kinase activity Relationships: is a type of lipid kinase activity [GO:0001727]; is a type of phosphotransferase activity, alcohol group as acceptor [GO:0016773] Subtypes: 1-phosphatidylinositol-3-phosphate 5-kinase activity [GO:0000285], 1-phosphatidylinositol 4-kinase activity [GO:0004430], 1-phosphatidylinositol-3-kinase activity [GO:0016303], 1-phosphatidylinositol-4-phosphate 5-kinase activity [GO:0016308], GO:0016309, 1-phosphatidylinositol-4-phosphate 3-kinase activity [GO:0035005], 1-phosphatidylinositol-4,5-bisphosphate 3-kinase activity [GO:0046934], 1-phosphatidylinositol-5-kinase activity [GO:0052810], 1-phosphatidylinositol-3-phosphate 4-kinase activity [GO:0052811]